{
  "term_label": "integrin complex",
  "term_id": "GO:0008305",
  "gene_name": "Integrin alpha-E",
  "gene": "UniProtKB:P38570",
  "gene_symbol": "ITGAE"
}